{
  "gene_symbol": "RING1",
  "term_id": "GO:0061630",
  "gene": "UniProtKB:Q06587",
  "gene_name": "E3 ubiquitin-protein ligase RING1",
  "term_label": "ubiquitin protein ligase activity"
}